stereocilium base [GO:0120044] (cellular component) Also known as: stereocilium taper Relationships: is a type of GO:0110165; is part of GO:0032420 Definition: The tapered base of the stereocilium adjacent to where it joins the hair cell body. This region contains a rootlet comprised of bundled actin filaments which spans the joint and stabilizes the stereocilium. References: PMID:20170899 Sources: GOC:krc